{
  "gene_symbol": "SNX8",
  "term_label": "intracellular protein transport",
  "gene_name": "Sorting nexin-8",
  "gene": "UniProtKB:Q9Y5X2",
  "term_id": "GO:0006886"
}